{
  "term_label": "intracellular copper ion homeostasis",
  "gene": "UniProtKB:Q04656",
  "gene_name": "Copper-transporting ATPase 1",
  "gene_symbol": "ATP7A",
  "term_id": "GO:0006878"
}